{
  "gene_name": "Tripartite motif-containing protein 26",
  "gene_symbol": "TRIM26",
  "term_id": "GO:0046597",
  "gene": "UniProtKB:Q12899",
  "term_label": "host-mediated suppression of symbiont invasion"
}